{
  "gene_name": "Multimerin-2",
  "gene": "UniProtKB:Q9H8L6",
  "gene_symbol": "MMRN2",
  "term_id": "UNKNOWN:0003",
  "term_label": "Unknown cellular component"
}